triglyceride transfer activity [GO:0140344] (MF) Relationships: is a type of lipid transfer activity [GO:0120013] Also known as: triglyceride carrier activity References: PMID:23475612 Definition: Directly binding to a triglyceride and delivering it either to an acceptor molecule or to a specific location.